iron sensor activity [GO:0140482] (molecular function) References: PMID:11956219, PMID:25806539 Relationships: is a type of metal ion sensor activity [GO:0140784] Definition: Binding to and responding, e.g. by conformational change, to changes in the cellular level of iron.